{
  "gene_name": "Zinc finger protein neuro-d4",
  "gene": "UniProtKB:Q92782",
  "term_id": "GO:0003712",
  "gene_symbol": "DPF1",
  "term_label": "transcription coregulator activity"
}